Z-farnesyl diphosphate synthase activity [GO:0033850] (molecular function) Also known as: (Z)-farnesyl diphosphate synthase activity, geranyl-diphosphate:isopentenyl-diphosphate geranylcistransferase activity Relationships: is_a transferase activity, transferring alkyl or aryl (other than methyl) groups [GO:0016765] Definition: Catalysis of the reaction: geranyl diphosphate + isopentenyl diphosphate = 2-cis,6-trans-farnesyl diphosphate + diphosphate. Sources: EC:2.5.1.68, RHEA:23300